{
  "gene_name": "Melatonin-related receptor",
  "gene_symbol": "GPR50",
  "term_label": "plasma membrane",
  "gene": "UniProtKB:Q13585",
  "term_id": "GO:0005886"
}